BMP receptor binding [GO:0070700] (molecular function) Also known as: bone morphogenetic protein receptor binding Definition: Binding to a BMP receptor. Sources: GOC:BHF, GOC:vk Relationships: is_a GO:0070696